FNIP-folliculin RagC/D GAP [GO:1990877] (cellular component) Relationships: is a type of GTPase activator complex [GO:1902773] Definition: A heterodimeric complex that functions as a GTPase-Activating Protein (GAP) Complex for members of the Rag family of GTPases. In the budding yeast, this complex contains Lst4 and Lst7, while the orthologous mammalian complex contains follicular (FLCN) and either follicular interacting protein 1 (FNIP1) or FNIP2. References: PMID:24095279, PMID:26387955, PMID:34805795 Sources: GOC:rn Also known as: BFC complex, FLCN-FNIP1 complex, FLCN-FNIP2 complex, FNIP-Folliculin RagC/D GAP complex, Lst4-Lst7 complex